{
  "gene_symbol": "KBTBD13",
  "term_label": "relaxation of skeletal muscle",
  "term_id": "GO:0090076",
  "gene": "UniProtKB:C9JR72",
  "gene_name": "Kelch repeat and BTB domain-containing protein 13"
}